somatotropin secreting cell differentiation [GO:0060126] (biological process) Definition: The process in which a relatively unspecialized cell acquires specialized structural and/or functional features of a somatotropin secreting cell. A somatotropin secreting cell is an acidophilic cell of the anterior pituitary that produces growth hormone, somatotropin. Also known as: growth hormone secreting cell differentiation, somatotrophin secreting cell differentiation, somatotrope differentiation, somatotroph differentiation, somatotropic cell differentiation, somatrophic cell differentiation Sources: GOC:dph Relationships: is a type of cell differentiation [GO:0030154]; is part of adenohypophysis development [GO:0021984]